{
  "gene_name": "Corepressor interacting with RBPJ 1",
  "term_id": "GO:0045892",
  "term_label": "negative regulation of DNA-templated transcription",
  "gene_symbol": "CIR1",
  "gene": "UniProtKB:Q86X95"
}